{
  "term_label": "Unknown biological process",
  "term_id": "UNKNOWN:0002",
  "gene_name": "DNA damage-induced apoptosis suppressor protein",
  "gene": "UniProtKB:Q8IXT1",
  "gene_symbol": "DDIAS"
}